{
  "gene": "UniProtKB:P61916",
  "gene_symbol": "NPC2",
  "term_label": "cholesterol efflux",
  "gene_name": "NPC intracellular cholesterol transporter 2",
  "term_id": "GO:0033344"
}